carnosine N-methyltransferase activity [GO:0030735] (molecular function) Sources: EC:2.1.1.22, RHEA:14205 Relationships: is a type of S-adenosylmethionine-dependent methyltransferase activity [GO:0008757] Also known as: S-adenosyl-L-methionine:carnosine N-methyltransferase activity Definition: Catalysis of the reaction: S-adenosyl-L-methionine + carnosine = S-adenosyl-L-homocysteine + anserine + H+.